lysine biosynthetic process via aminoadipic acid [GO:0019878] (biological process) Regulation: regulated by regulation of lysine biosynthetic process via aminoadipic acid [GO:1902986]; negatively regulated by negative regulation of lysine biosynthetic process via aminoadipic acid [GO:1902987] Relationships: is a type of lysine biosynthetic process [GO:0009085] Also known as: lysine anabolism via aminoadipic acid, lysine biosynthesis, aminoadipic acid pathway, lysine biosynthesis, aminoadipic pathway, lysine biosynthetic process, aminoadipic acid pathway, lysine biosynthetic process, aminoadipic pathway, lysine formation via aminoadipic acid, lysine synthesis via aminoadipic acid Definition: The chemical reactions and pathways resulting in the formation of lysine by the aminoadipic pathway. Sources: GOC:go_curators Subtypes: lysine biosynthetic process via alpha-aminoadipate and saccharopine [GO:0051975], lysine biosynthetic process via alpha-aminoadipate and N2-acetyl-alpha-aminoadipate [GO:0051976]